macrophage differentiation [GO:0030225] (biological process) Definition: The process in which a relatively unspecialized monocyte acquires the specialized features of a macrophage. Also known as: macrophage cell differentiation Regulation: regulated by regulation of macrophage differentiation [GO:0045649]; negatively regulated by negative regulation of macrophage differentiation [GO:0045650]; positively regulated by positive regulation of macrophage differentiation [GO:0045651] Relationships: is a type of myeloid leukocyte differentiation [GO:0002573]; is a type of mononuclear cell differentiation [GO:1903131] Sources: GOC:add, ISBN:0781735149 Subtypes: microglia differentiation [GO:0014004]